{
  "gene": "UniProtKB:P0CG37",
  "term_label": "cell surface",
  "gene_symbol": "CFC1",
  "gene_name": "Cryptic protein",
  "term_id": "GO:0009986"
}